{
  "term_id": "GO:0005615",
  "gene_symbol": "OMD",
  "term_label": "extracellular space",
  "gene": "UniProtKB:Q99983",
  "gene_name": "Osteomodulin"
}